external side of fungal-type cell wall [GO:0070263] (cellular component) Relationships: is a type of external side of cell wall [GO:0010339]; is part of fungal-type cell wall [GO:0009277] Definition: The side of the fungal-type cell wall that is opposite to the side that faces the cell and its contents. Sources: GOC:mah